{
  "term_label": "DNA-binding transcription factor activity, RNA polymerase II-specific",
  "term_id": "GO:0000981",
  "gene_symbol": "ISL2",
  "gene": "UniProtKB:Q96A47",
  "gene_name": "Insulin gene enhancer protein ISL-2"
}